FADH2 metabolic process [GO:0006746] (biological process) Relationships: is a type of flavin adenine dinucleotide metabolic process [GO:0072387] Definition: The chemical reactions and pathways involving the reduced form of flavin adenine dinucleotide. Sources: GOC:ai Also known as: FADH2 metabolism, reduced flavin adenine dinucleotide metabolic process